{
  "gene_name": "Zinc transporter ZIP4",
  "gene": "UniProtKB:Q6P5W5",
  "term_label": "intracellular monoatomic cation homeostasis",
  "term_id": "GO:0030003",
  "gene_symbol": "SLC39A4"
}